{
  "term_label": "Unknown molecular function",
  "term_id": "UNKNOWN:0001",
  "gene_symbol": "IGLV7-43",
  "gene": "UniProtKB:P04211",
  "gene_name": "Immunoglobulin lambda variable 7-43"
}